{
  "term_id": "GO:0019888",
  "gene_name": "Serine_threonine-protein phosphatase 6 regulatory subunit 3",
  "term_label": "protein phosphatase regulator activity",
  "gene_symbol": "PPP6R3",
  "gene": "UniProtKB:Q5H9R7"
}